{
  "gene_symbol": "CCIN",
  "term_label": "cytoplasm",
  "gene_name": "Calicin",
  "gene": "UniProtKB:Q13939",
  "term_id": "GO:0005737"
}